regulation of nodal signaling pathway [GO:1900107] (biological process) Definition: Any process that modulates the frequency, rate or extent of nodal signaling pathway. Relationships: is a type of regulation of activin receptor signaling pathway [GO:0032925]; regulates nodal signaling pathway [GO:0038092] Sources: GOC:BHF, GOC:TermGenie, GOC:vk Subtypes: positive regulation of nodal signaling pathway [GO:0141092], negative regulation of nodal signaling pathway [GO:1900108] Also known as: regulation of nodal signaling, regulation of nodal signalling pathway